{
  "gene_name": "Calcium_calmodulin-dependent protein kinase type II subunit delta",
  "term_label": "regulation of protein localization to plasma membrane",
  "gene_symbol": "CAMK2D",
  "gene": "UniProtKB:Q13557",
  "term_id": "GO:1903076"
}